{
  "gene_symbol": "PRDM10",
  "gene": "UniProtKB:Q9NQV6",
  "gene_name": "PR domain zinc finger protein 10",
  "term_label": "DNA-binding transcription factor activity",
  "term_id": "GO:0003700"
}